{
  "term_label": "Unknown biological process",
  "gene_name": "Small ribosomal subunit protein eS26",
  "gene": "UniProtKB:P62854",
  "gene_symbol": "RPS26",
  "term_id": "UNKNOWN:0002"
}